saccharopine dehydrogenase (NAD+, L-lysine-forming) activity [GO:0004754] (MF) Definition: Catalysis of the reaction: L-saccharopine + H2O + NAD+ = 2-oxoglutarate + L-lysine + H+ + NADH. Relationships: is a type of saccharopine dehydrogenase activity [GO:0004753] Also known as: 6-N-(L-1,3-dicarboxypropyl)-L-lysine:NAD+ oxidoreductase (L-lysine-forming), N6-(L-1,3-dicarboxypropyl)-L-lysine:NAD+ oxidoreductase (L-lysine-forming), N6-(glutar-2-yl)-L-lysine:NAD oxidoreductase (L-lysine-forming), dehydrogenase, saccharopine (nicotinamide adenine dinucleotide, lysine forming), epsilon-N-(L-glutaryl-2)-L-lysine:NAD oxidoreductase (L-lysine forming) Sources: EC:1.5.1.7, RHEA:12440